{
  "gene_name": "Zinc finger protein 212",
  "gene": "UniProtKB:Q9UDV6",
  "term_label": "regulation of transcription by RNA polymerase II",
  "term_id": "GO:0006357",
  "gene_symbol": "ZNF212"
}